{
  "term_label": "Unknown cellular component",
  "gene_name": "Microtubule-associated tyrosine carboxypeptidase 1",
  "gene_symbol": "MATCAP1",
  "term_id": "UNKNOWN:0003",
  "gene": "UniProtKB:Q68EN5"
}